{
  "gene_name": "Leydig cell tumor 10 kDa protein homolog",
  "gene_symbol": "C19orf53",
  "gene": "UniProtKB:Q9UNZ5",
  "term_label": "Unknown molecular function",
  "term_id": "UNKNOWN:0001"
}